Weibel-Palade body [GO:0033093] (cellular component) Relationships: is a type of GO:0030136; is a type of GO:0030141 Definition: A large, elongated, rod-shaped secretory granule characteristic of vascular endothelial cells that contain a number of structurally and functionally distinct proteins, of which the best characterized are von Willebrand factor (VWF) and P-selectin. Weibel-Palade bodies are formed from the trans-Golgi network in a process that depends on VWF, which is densely packed in a highly organized manner, and on coat proteins that remain associated with the granules. Upon cell stimulation, regulated exocytosis releases the contained proteins to the cell surface, where they act in the recruitment of platelets and leukocytes and in inflammatory and vasoactive responses. References: PMID:11935287, PMID:16087708